{
  "term_id": "GO:0005549",
  "gene_symbol": "OR13G1",
  "gene": "UniProtKB:Q8NGZ3",
  "gene_name": "Olfactory receptor 13G1",
  "term_label": "odorant binding"
}